vasoconstriction of artery involved in chemoreceptor response to lowering of systemic arterial blood pressure [GO:0002012] (biological process) Subtypes: GO:0003042, vasoconstriction of artery involved in aortic body chemoreceptor response to lowering of systemic arterial blood pressure [GO:0003043] Definition: A process that is triggered by vasomotor excitation and results in a decrease in the diameter of an artery during the chemoreceptor response to decreased blood pressure. Relationships: is a type of positive regulation of systemic arterial blood pressure [GO:0003084]; is a type of vasoconstriction [GO:0042310]; BFO_0000050 GO:0001979 Sources: GOC:dph, GOC:mtg_cardio